{
  "gene": "UniProtKB:Q9NTM9",
  "gene_name": "Copper homeostasis protein cutC homolog",
  "term_id": "UNKNOWN:0003",
  "term_label": "Unknown cellular component",
  "gene_symbol": "CUTC"
}